cerebral cortex neuron differentiation [GO:0021895] (biological process) Subtypes: Cajal-Retzius cell differentiation [GO:0021870], cerebral cortex GABAergic interneuron differentiation [GO:0021892], hippocampal interneuron differentiation [GO:0097410], GO:0097432, Meynert cell differentiation [GO:1905270] Sources: GOC:cls, GOC:dgh, GOC:dph, GOC:jid, GO_REF:0000021 Relationships: is a type of forebrain neuron differentiation [GO:0021879] Definition: The process in which a relatively unspecialized cell acquires specialized features of a neuron residing in the cerebral cortex.